{
  "term_label": "Unknown biological process",
  "gene_symbol": "LINC00470",
  "gene_name": "Putative uncharacterized protein encoded by LINC00470",
  "term_id": "UNKNOWN:0002",
  "gene": "UniProtKB:Q9BZP3"
}